{
  "gene_symbol": "TMEM132C",
  "term_id": "UNKNOWN:0001",
  "gene": "UniProtKB:Q8N3T6",
  "term_label": "Unknown molecular function",
  "gene_name": "Transmembrane protein 132C"
}